{
  "gene": "UniProtKB:Q14997",
  "gene_symbol": "PSME4",
  "term_id": "GO:0010499",
  "gene_name": "Proteasome activator complex subunit 4",
  "term_label": "proteasomal ubiquitin-independent protein catabolic process"
}